{
  "gene_name": "Heat shock 70 kDa protein 14",
  "term_label": "ATP hydrolysis activity",
  "gene": "UniProtKB:Q0VDF9",
  "term_id": "GO:0016887",
  "gene_symbol": "HSPA14"
}